cloacal gland development [GO:1904484] (biological process) Relationships: is a type of gland development [GO:0048732] References: PMID:18805421 Sources: GOC:TermGenie, GOC:mr, GO_REF:0000094 Definition: The process whose specific outcome is the progression of a cloacal gland over time, from its formation to the mature structure.